{
  "gene": "UniProtKB:Q9NRA0",
  "gene_symbol": "SPHK2",
  "gene_name": "Sphingosine kinase 2",
  "term_label": "sphingosine biosynthetic process",
  "term_id": "GO:0046512"
}